negative regulation of aldosterone secretion [GO:2000859] (biological process) Relationships: is a type of negative regulation of mineralocorticoid secretion [GO:2000856]; is a type of regulation of aldosterone secretion [GO:2000858]; negatively regulates aldosterone secretion [GO:0035932] Definition: Any process that stops, prevents or reduces the frequency, rate or extent of aldosterone secretion. Sources: GOC:sl